{
  "gene_name": "Cystatin-SN",
  "term_label": "vesicle",
  "gene_symbol": "CST1",
  "gene": "UniProtKB:P01037",
  "term_id": "GO:0031982"
}